{
  "term_label": "G protein-coupled receptor signaling pathway",
  "gene": "UniProtKB:P0DN78",
  "gene_name": "Medium-wave-sensitive opsin 3",
  "term_id": "GO:0007186",
  "gene_symbol": "OPN1MW3"
}